mRNA guanylyltransferase activity [GO:0004484] (molecular function) Sources: EC:2.7.7.50 Relationships: is a type of RNA guanylyltransferase activity [GO:0008192] Also known as: GTP:mRNA guanylyltransferase activity, GTP--RNA guanylyltransferase activity, mRNA capping enzyme activity, messenger RNA guanylyltransferase activity, protein lambda2 Definition: Catalysis of the reaction: GTP + (5')pp-Pur-mRNA = diphosphate + G(5')ppp-Pur-mRNA; G(5')ppp-Pur-mRNA is mRNA containing a guanosine residue linked 5' through three phosphates to the 5' position of the terminal residue.